oligosaccharyltransferase complex A [GO:0160226] (cellular component) Also known as: OST-A Relationships: is a type of GO:0008250 References: PMID:31831667, PMID:39509507 Definition: An oligosaccharyltransferase complex that contains STT3A as the catalytic subunit.